{
  "term_label": "negative regulation of t-circle formation",
  "gene_symbol": "RTEL1",
  "gene": "UniProtKB:Q9NZ71",
  "term_id": "GO:1904430",
  "gene_name": "Regulator of telomere elongation helicase 1"
}